{
  "gene": "UniProtKB:Q6IS14",
  "gene_name": "Eukaryotic translation initiation factor 5A-1-like",
  "term_label": "Unknown cellular component",
  "gene_symbol": "EIF5AL1",
  "term_id": "UNKNOWN:0003"
}